{
  "gene": "UniProtKB:B7ZW38",
  "gene_symbol": "HNRNPCL3",
  "gene_name": "Heterogeneous nuclear ribonucleoprotein C-like 3",
  "term_id": "UNKNOWN:0002",
  "term_label": "Unknown biological process"
}